{
  "gene": "UniProtKB:Q96N68",
  "term_label": "Unknown biological process",
  "gene_symbol": "C18orf15",
  "gene_name": "Putative uncharacterized protein C18orf15",
  "term_id": "UNKNOWN:0002"
}